{
  "term_label": "beta-catenin binding",
  "term_id": "GO:0008013",
  "gene_name": "Cadherin-15",
  "gene_symbol": "CDH15",
  "gene": "UniProtKB:P55291"
}